{
  "gene_symbol": "LRRK2",
  "gene_name": "Leucine-rich repeat serine_threonine-protein kinase 2",
  "term_label": "Golgi organization",
  "gene": "UniProtKB:Q5S007",
  "term_id": "GO:0007030"
}